negative regulation of ERBB4 signaling pathway [GO:0120154] (biological process) Definition: Any process that stops, prevents or reduces the frequency, rate or extent of ERBB4 signaling pathway. References: PMID:15219672 Relationships: is a type of negative regulation of ERBB signaling pathway [GO:1901185]; negatively regulates GO:0038130